{
  "gene_symbol": "GSG1L2",
  "gene": "UniProtKB:A8MUP6",
  "term_label": "plasma membrane",
  "gene_name": "Germ cell-specific gene 1-like protein 2",
  "term_id": "GO:0005886"
}